{
  "gene_symbol": "INSYN2A",
  "gene": "UniProtKB:Q6ZSG2",
  "term_id": "UNKNOWN:0001",
  "term_label": "Unknown molecular function",
  "gene_name": "Inhibitory synaptic factor 2A"
}